{
  "gene_name": "Blood group Rh(D) polypeptide",
  "term_id": "GO:0097272",
  "term_label": "ammonium homeostasis",
  "gene_symbol": "RHD",
  "gene": "UniProtKB:Q02161"
}